{
  "term_label": "endopeptidase activity",
  "gene_symbol": "PSMB7",
  "gene": "UniProtKB:Q99436",
  "gene_name": "Proteasome subunit beta type-7",
  "term_id": "GO:0004175"
}